mature chylomicron [GO:0034359] (CC) Definition: A chylomicron that contains apolipoprotein C2 (APOC2), a cofactor for lipoprotein lipase (LPL) activity, and has a mean diameter of 500 nm and density of 0.95g/ml. Mature chylomicron particles transport exogenous (dietary) lipids from the intestines to other body tissues, via the blood and lymph. Relationships: is a type of GO:0042627 Sources: GOC:BHF, GOC:expert_pt, GOC:mah, GOC:rl